{
  "gene": "UniProtKB:Q8NFU5",
  "gene_symbol": "IPMK",
  "gene_name": "Inositol polyphosphate multikinase",
  "term_id": "GO:0032958",
  "term_label": "inositol phosphate biosynthetic process"
}